{
  "gene_symbol": "C7orf25",
  "gene": "UniProtKB:Q9BPX7",
  "term_label": "Unknown biological process",
  "gene_name": "UPF0415 protein C7orf25",
  "term_id": "UNKNOWN:0002"
}